{
  "term_id": "GO:0003729",
  "gene": "UniProtKB:A6NFN3",
  "gene_name": "RNA binding protein fox-1 homolog 3",
  "term_label": "mRNA binding",
  "gene_symbol": "RBFOX3"
}